glucose-6-phosphatase activity [GO:0004346] (molecular function) Relationships: is a type of sugar-terminal-phosphatase activity [GO:0050309] Definition: Catalysis of the reaction: D-glucopyranose 6-phosphate + H2O = D-glucose + phosphate. D-glucopyranose is also known as D-glucose 6-phosphate. Also known as: D-glucose-6-phosphate phosphohydrolase activity, glucose 6-phosphate phosphatase activity Sources: EC:3.1.3.9, RHEA:16689